propan-2-ol biosynthetic process [GO:1902640] (biological process) References: PMID:16346237 Sources: GOC:TermGenie, GOC:mengo_curators, GO_REF:0000068 Relationships: is a type of secondary alcohol biosynthetic process [GO:1902653]; is a type of GO:1903175 Definition: The chemical reactions and pathways resulting in the formation of propan-2-ol. Also known as: Isopropanol biosynthetic process, Isopropyl alcohol biosynthetic process, propan-2-ol anabolism, propan-2-ol biosynthesis, propan-2-ol formation, propan-2-ol synthesis